maintenance of protein location to spindle pole body [GO:0071990] (biological process) Definition: Any process in which a protein is maintained in a specific location at the spindle pole body, and is prevented from moving elsewhere. Relationships: is a type of cell cycle process [GO:0022402]; is a type of maintenance of protein localization in organelle [GO:0072595]; is part of GO:0051300; is part of GO:0071988; occurs in spindle pole body [GO:0005816] Sources: GOC:mah, GOC:vw Also known as: maintenance of protein location at spindle pole body, maintenance of protein location in spindle pole body